{
  "gene_symbol": "SLC6A6",
  "gene_name": "Sodium- and chloride-dependent taurine transporter",
  "term_id": "GO:0005886",
  "gene": "UniProtKB:P31641",
  "term_label": "plasma membrane"
}